{
  "gene_symbol": "OR2C1",
  "gene": "UniProtKB:O95371",
  "term_id": "GO:0004984",
  "gene_name": "Olfactory receptor 2C1",
  "term_label": "olfactory receptor activity"
}